{
  "gene_name": "Gamma-glutamylcyclotransferase",
  "gene": "UniProtKB:O75223",
  "term_label": "Unknown cellular component",
  "term_id": "UNKNOWN:0003",
  "gene_symbol": "GGCT"
}